wobble position ribose methylation [GO:0002130] (biological process) Sources: GOC:hjd, ISBN:155581073X Relationships: is a type of tRNA nucleoside ribose methylation [GO:0002128] Definition: The process in which the ribose base of the nucleotide at position 34 in the anticodon of a tRNA is post-transcriptionally methylated at the 2'O position. Subtypes: wobble position guanine ribose methylation [GO:0002129], wobble position cytosine ribose methylation [GO:0002131], wobble position uridine ribose methylation [GO:0002132]